1-hydroxy-2-naphthoate hydroxylase activity [GO:0018637] (molecular function) References: PMID:20727010, PMID:21545490 Sources: EC:1.14.13.135, UM-BBD_reactionID:r0491 Relationships: is a type of oxidoreductase activity, acting on paired donors, with incorporation or reduction of molecular oxygen, NAD(P)H as one donor, and incorporation of one atom of oxygen [GO:0016709] Definition: Catalysis of the reaction: 1-hydroxy-2-naphthoate + O2 + NAD(P)H + 2 H+ = NAD(P)+ + H2O + CO2 + 1,2-dihydroxynaphthalene.